{
  "term_label": "early endosome",
  "gene_name": "Pleckstrin homology domain-containing family F member 2",
  "gene": "UniProtKB:Q9H8W4",
  "gene_symbol": "PLEKHF2",
  "term_id": "GO:0005769"
}